{
  "term_id": "UNKNOWN:0001",
  "gene_symbol": "NOG",
  "gene": "UniProtKB:Q13253",
  "gene_name": "Noggin",
  "term_label": "Unknown molecular function"
}